lactonohydrolase activity [GO:0046573] (molecular function) Definition: Catalysis of the hydrolysis of lactone rings (intramolecular cyclic esters) to produce a hydroxyl group and a carboxyl group. Subtypes: 5-valerolactone hydrolase activity [GO:0055042], GO:0102007 References: PMID:11640988 Relationships: is a type of carboxylic ester hydrolase activity [GO:0052689]